{
  "term_id": "UNKNOWN:0003",
  "gene_name": "Protein FAM90A19",
  "gene": "UniProtKB:P0DV76",
  "term_label": "Unknown cellular component",
  "gene_symbol": "FAM90A19"
}